{
  "term_label": "nicotinate riboside kinase activity",
  "gene_symbol": "NMRK2",
  "gene": "UniProtKB:Q9NPI5",
  "term_id": "GO:0061769",
  "gene_name": "Nicotinamide riboside kinase 2"
}